{
  "gene_name": "Alpha-mannosidase 2C1",
  "gene": "UniProtKB:Q9NTJ4",
  "gene_symbol": "MAN2C1",
  "term_label": "alpha-mannosidase activity",
  "term_id": "GO:0004559"
}